hemoglobin metabolic process [GO:0020027] (biological process) Definition: The chemical reactions and pathways involving hemoglobin, including its uptake and utilization. Relationships: is a type of protein metabolic process [GO:0019538] Also known as: haemoglobin metabolic process, haemoglobin metabolism, hemoglobin metabolism Subtypes: GO:0042540, hemoglobin biosynthetic process [GO:0042541] Sources: GOC:go_curators, GOC:jl